kidney mesenchyme morphogenesis [GO:0072131] (biological process) Subtypes: GO:0061221, GO:0072133, nephrogenic mesenchyme morphogenesis [GO:0072134] Definition: The process in which the anatomical structures of a kidney mesenchymal tissue are generated and organized. Kidney mesenchyme is the tissue made up of loosely connected mesenchymal cells in the kidney. Relationships: is a type of mesenchyme morphogenesis [GO:0072132]; is part of GO:0072074 Sources: GOC:mtg_kidney_jan10